{
  "term_id": "GO:0009986",
  "gene_name": "Signal peptide, CUB and EGF-like domain-containing protein 3",
  "gene_symbol": "SCUBE3",
  "term_label": "cell surface",
  "gene": "UniProtKB:Q8IX30"
}